regulation of platelet activation [GO:0010543] (BP) Relationships: is a type of GO:0050865; regulates platelet activation [GO:0030168] Subtypes: negative regulation of platelet activation [GO:0010544], positive regulation of platelet activation [GO:0010572], regulation of platelet aggregation [GO:0090330] Sources: GOC:BHF, GOC:dph, GOC:tb Definition: Any process that modulates the rate or frequency of platelet activation. Platelet activation is a series of progressive, overlapping events triggered by exposure of the platelets to subendothelial tissue.